regulation of synapse structure or activity [GO:0050803] (biological process) Relationships: is a type of regulation of biological quality [GO:0065008] Sources: GOC:ai Definition: Any process that modulates the physical form or the activity of a synapse, the junction between a neuron and a target (neuron, muscle, or secretory cell).